regulation of fatty acid beta-oxidation using acyl-CoA dehydrogenase [GO:1904735] (biological process) Relationships: is a type of regulation of fatty acid beta-oxidation [GO:0031998]; regulates fatty acid beta-oxidation using acyl-CoA dehydrogenase [GO:0033539] Subtypes: negative regulation of fatty acid beta-oxidation using acyl-CoA dehydrogenase [GO:1904736], positive regulation of fatty acid beta-oxidation using acyl-CoA dehydrogenase [GO:1904737] Definition: Any process that modulates the frequency, rate or extent of fatty acid beta-oxidation using acyl-CoA dehydrogenase. References: PMID:25416781 Sources: GOC:TermGenie, GO_REF:0000058